anaerobic glycine catabolic process [GO:0019669] (BP) Also known as: glycine fermentation Relationships: is a type of glycine catabolic process [GO:0006546]; is a type of anaerobic amino acid catabolic process [GO:0019665]; is part of GO:0019668 Sources: GOC:jl Definition: The anaerobic chemical reactions and pathways resulting in the breakdown of glycine, yielding energy in the form of ATP.